{
  "gene": "UniProtKB:Q9UG63",
  "term_id": "UNKNOWN:0003",
  "term_label": "Unknown cellular component",
  "gene_name": "ATP-binding cassette sub-family F member 2",
  "gene_symbol": "ABCF2"
}